{
  "gene_symbol": "MSS51",
  "term_label": "Unknown cellular component",
  "gene": "UniProtKB:Q4VC12",
  "term_id": "UNKNOWN:0003",
  "gene_name": "Putative protein MSS51 homolog, mitochondrial"
}